extrinsic component of cell outer membrane [GO:0031244] (cellular component) Also known as: extrinsic to cell outer membrane Subtypes: extrinsic component of external side of cell outer membrane [GO:0031242], extrinsic component of periplasmic side of cell outer membrane [GO:0031245], GO:0036420 Relationships: is a type of extrinsic component of membrane [GO:0019898]; is part of cell outer membrane [GO:0009279] Definition: The component of the cell outer membrane consisting of gene products and protein complexes that are loosely bound to one of its surfaces, but not integrated into the hydrophobic region. Sources: GOC:dos, GOC:mah, GOC:mtg_sensu